{
  "term_id": "GO:0005886",
  "gene": "UniProtKB:P40967",
  "gene_name": "Melanocyte protein PMEL",
  "term_label": "plasma membrane",
  "gene_symbol": "PMEL"
}